{
  "gene_name": "Plastin-3",
  "gene": "UniProtKB:P13797",
  "gene_symbol": "PLS3",
  "term_id": "GO:0032432",
  "term_label": "actin filament bundle"
}